{
  "gene_name": "Properdin",
  "gene_symbol": "CFP",
  "term_id": "UNKNOWN:0001",
  "term_label": "Unknown molecular function",
  "gene": "UniProtKB:P27918"
}